mast cell secretagogue receptor activity [GO:1990595] (molecular function) References: PMID:25517090 Sources: GOC:sp Relationships: is a type of G protein-coupled receptor activity [GO:0004930] Definition: Combining with basic secretagogues to initiate pseudo-allergic reactions in mast cells.